{
  "gene_symbol": "SLC25A12",
  "term_id": "GO:0015183",
  "gene": "UniProtKB:O75746",
  "term_label": "L-aspartate transmembrane transporter activity",
  "gene_name": "Electrogenic aspartate_glutamate antiporter SLC25A12, mitochondrial"
}